{
  "term_label": "Rab geranylgeranyltransferase activity",
  "term_id": "GO:0004663",
  "gene_symbol": "RABGGTB",
  "gene_name": "Geranylgeranyl transferase type-2 subunit beta",
  "gene": "UniProtKB:P53611"
}